{
  "term_id": "UNKNOWN:0003",
  "gene_symbol": "HMHB1",
  "gene_name": "Minor histocompatibility protein HB-1",
  "gene": "UniProtKB:O97980",
  "term_label": "Unknown cellular component"
}